regulation of protein localization to phagocytic vesicle [GO:1905169] (biological process) Definition: Any process that modulates the frequency, rate or extent of protein localization to phagocytic vesicle. Subtypes: negative regulation of protein localization to phagocytic vesicle [GO:1905170], positive regulation of protein localization to phagocytic vesicle [GO:1905171] Sources: GOC:PARL, GOC:TermGenie, GOC:bf, GO_REF:0000058 Also known as: regulation of protein localisation in phagocytic vesicle, regulation of protein localisation to phagocytic vesicle, regulation of protein localisation to phagosome, regulation of protein localization in phagocytic vesicle, regulation of protein recruitment to phagosome Relationships: is a type of regulation of protein localization [GO:0032880]; regulates GO:1905161